urate-ribonucleotide phosphorylase activity [GO:0050384] (molecular function) Definition: Catalysis of the reaction: 3-(beta-D-ribofuranosyl)uric acid + phosphate = alpha-D-ribose 1-phosphate + H+ + urate. Sources: EC:2.4.2.16, RHEA:13909 Relationships: is a type of pentosyltransferase activity [GO:0016763] Also known as: UAR phosphorylase activity, urate-ribonucleotide:phosphate D-ribosyltransferase activity, urate-ribonucleotide:phosphate alpha-D-ribosyltransferase activity